{
  "gene_name": "Branched-chain-amino-acid aminotransferase, cytosolic",
  "term_id": "GO:0004084",
  "gene_symbol": "BCAT1",
  "gene": "UniProtKB:P54687",
  "term_label": "branched-chain-amino-acid transaminase activity"
}